{
  "gene": "UniProtKB:Q16612",
  "gene_symbol": "NREP",
  "gene_name": "Neuronal regeneration-related protein",
  "term_id": "UNKNOWN:0001",
  "term_label": "Unknown molecular function"
}